{
  "term_label": "plasma membrane",
  "term_id": "GO:0005886",
  "gene_symbol": "PCDH11Y",
  "gene": "UniProtKB:Q9BZA8",
  "gene_name": "Protocadherin-11 Y-linked"
}